{
  "term_id": "UNKNOWN:0003",
  "gene_name": "Immunoglobulin heavy variable 2-70",
  "gene": "UniProtKB:P01814",
  "term_label": "Unknown cellular component",
  "gene_symbol": "IGHV2-70"
}